{
  "gene_name": "Putative uncharacterized protein FLJ11871",
  "gene_symbol": "Q9HAA7",
  "gene": "UniProtKB:Q9HAA7",
  "term_label": "Unknown molecular function",
  "term_id": "UNKNOWN:0001"
}